{
  "gene_name": "Transcription factor GATA-5",
  "term_id": "GO:0000978",
  "gene_symbol": "GATA5",
  "term_label": "RNA polymerase II cis-regulatory region sequence-specific DNA binding",
  "gene": "UniProtKB:Q9BWX5"
}